UAU codon-amino acid adaptor activity [GO:0033409] (molecular function) Definition: A triplet codon-amino acid adaptor activity that recognizes a UAU codon. Also known as: TAT codon-amino acid adaptor activity, tyrosine tRNA Sources: GOC:mah Relationships: is a type of triplet codon-amino acid adaptor activity [GO:0030533] Note: Note that in the standard genetic code, TAT codes for tyrosine.